{
  "term_label": "regulation of release of sequestered calcium ion into cytosol by sarcoplasmic reticulum",
  "gene_symbol": "CALM2",
  "gene_name": "Calmodulin-2",
  "gene": "UniProtKB:P0DP24",
  "term_id": "GO:0010880"
}